Cdc50p-Drs2p complex [GO:1990530] (cellular component) Definition: A protein complex that functions as a phospholipid-translocating P-Type ATPase. In budding yeast, this complex consists of Cdc50p and Drs2p proteins, and is involved in the trafficking of transport vesicles between the late Golgi and the early endosome. References: PMID:15090616, PMID:22234261 Sources: GOC:rb Relationships: is a type of phospholipid-translocating ATPase complex [GO:1990531]